{
  "term_id": "GO:0005615",
  "gene": "UniProtKB:P12645",
  "gene_symbol": "BMP3",
  "gene_name": "Bone morphogenetic protein 3",
  "term_label": "extracellular space"
}